{
  "term_id": "GO:0038023",
  "gene_name": "Cell surface glycoprotein CD200 receptor 1",
  "gene_symbol": "CD200R1",
  "gene": "UniProtKB:Q8TD46",
  "term_label": "signaling receptor activity"
}